iodide transmembrane transport [GO:1904200] (biological process) Definition: The process in which iodide is transported across a membrane. References: PMID:20392814 Sources: GOC:TermGenie, GO_REF:0000069 Regulation: regulated by regulation of iodide transmembrane transport [GO:1904212]; negatively regulated by negative regulation of iodide transmembrane transport [GO:1904213]; positively regulated by positive regulation of iodide transmembrane transport [GO:1904214] Relationships: is a type of iodide transport [GO:0015705]; is a type of GO:0098656